{
  "gene": "UniProtKB:Q8NGR3",
  "term_id": "GO:0016020",
  "term_label": "membrane",
  "gene_symbol": "OR1K1",
  "gene_name": "Olfactory receptor 1K1"
}